atrial cardiac muscle cell to AV node cell communication by electrical coupling [GO:0086044] (biological process) Sources: GOC:BHF, GOC:mtg_cardiac_conduct_nov11 Relationships: is a type of cell communication by electrical coupling involved in cardiac conduction [GO:0086064]; is a type of atrial cardiac muscle cell to AV node cell communication [GO:0086066] Also known as: atrial cardiomyocyte to AV node cell communication by electrical coupling, atrial cardiomyocyte to atrioventricular node cell communication by electrical coupling Definition: The process that mediates signaling interactions between an atrial cardiomyocyte and an AV node cell by transfer of current between their adjacent cytoplasms via intercellular protein channels.